{
  "term_label": "heme binding",
  "gene_name": "Transmembrane reductase CYB561D2",
  "gene_symbol": "CYB561D2",
  "gene": "UniProtKB:O14569",
  "term_id": "GO:0020037"
}